phragmosome [GO:0009525] (cellular component) Relationships: is a type of cellular anatomical structure [GO:0110165]; BFO_0000050 cytoplasm [GO:0005737] Definition: A flattened membranous vesicle containing cell wall components. Sources: ISBN:0943088399